{
  "term_label": "cytoplasm",
  "gene_symbol": "STAT2",
  "gene": "UniProtKB:P52630",
  "gene_name": "Signal transducer and activator of transcription 2",
  "term_id": "GO:0005737"
}